{
  "term_id": "GO:0098794",
  "gene_symbol": "GABRG3",
  "term_label": "postsynapse",
  "gene": "UniProtKB:Q99928",
  "gene_name": "Gamma-aminobutyric acid receptor subunit gamma-3"
}